{
  "gene_name": "Forkhead box protein P2",
  "gene": "UniProtKB:O15409",
  "gene_symbol": "FOXP2",
  "term_id": "GO:0007519",
  "term_label": "skeletal muscle tissue development"
}